metanephric distal tubule development [GO:0072235] (biological process) Definition: The process whose specific outcome is the progression of the metanephric distal tubule over time, from its formation to the mature structure. The metanephric distal tubule is a metanephric nephron tubule that begins at the metanephric macula densa and extends to the metanephric connecting tubule. Sources: GOC:mtg_kidney_jan10 Relationships: is a type of distal tubule development [GO:0072017]; is a type of metanephric nephron tubule development [GO:0072234]